negative regulation of excitatory synapse pruning [GO:1905811] (biological process) Definition: Any process that stops, prevents or reduces the frequency, rate or extent of excitatory synapse pruning. Also known as: regulation of synapse clearance, regulation of synapse disassembly, regulation of synapse elimination, regulation of synapse removal, down regulation of excitatory synapse disassembly, down-regulation of excitatory synapse disassembly, downregulation of excitatory synapse disassembly, inhibition of excitatory synapse disassembly Relationships: is a type of GO:1905807; is_a GO:1905810; negatively regulates excitatory synapse pruning [GO:1905805] References: PMID:27779093 Sources: GOC:TermGenie, GO_REF:0000058